{
  "gene": "UniProtKB:Q86V97",
  "gene_symbol": "KBTBD6",
  "gene_name": "Kelch repeat and BTB domain-containing protein 6",
  "term_id": "GO:0043161",
  "term_label": "proteasome-mediated ubiquitin-dependent protein catabolic process"
}